{
  "term_label": "mitochondrial respiratory chain complex I assembly",
  "term_id": "GO:0032981",
  "gene_name": "Cytochrome c oxidase assembly factor 1 homolog",
  "gene": "UniProtKB:Q9GZY4",
  "gene_symbol": "COA1"
}